positive regulation of (R)-carnitine transmembrane transport [GO:1902274] (biological process) Also known as: up regulation of (R)-carnitine transmembrane transport, up-regulation of (R)-carnitine transmembrane transport, upregulation of (R)-carnitine transmembrane transport, activation of (R)-carnitine transmembrane transport Relationships: is a type of positive regulation of transmembrane transport [GO:0034764]; is a type of regulation of (R)-carnitine transmembrane transport [GO:1902272]; positively regulates (R)-carnitine transmembrane transport [GO:1902270] References: PMID:23755272 Sources: GOC:TermGenie Definition: Any process that activates or increases the frequency, rate or extent of (R)-carnitine transmembrane transport.